alcohol dehydrogenase (NADP+) activity [GO:0008106] (molecular function) Sources: EC:1.1.1.2 Also known as: NADP-aldehyde reductase activity, alcohol:NADP dehydrogenase activity, aldehyde reductase (NADPH) activity Definition: Catalysis of the reaction: an alcohol + NADP+ = an aldehyde or ketone + NADPH + H+. Relationships: is a type of GO:0018455 Subtypes: aldose reductase (NADPH) activity [GO:0004032], carbonyl reductase (NADPH) activity [GO:0004090], GO:0032018, pyridoxine 4-dehydrogenase (NADP+) activity [GO:0050236], all-trans-retinol dehydrogenase (NADP+) activity [GO:0052650], 3-methylbutanal reductase (NADPH) activity [GO:0052675], 11-cis-retinol dehydrogenase (NADP+) activity [GO:0102354]